{
  "gene": "UniProtKB:Q96RL6",
  "gene_symbol": "SIGLEC11",
  "term_id": "GO:0007155",
  "gene_name": "Sialic acid-binding Ig-like lectin 11",
  "term_label": "cell adhesion"
}